{
  "gene_name": "Dual specificity protein kinase TTK",
  "gene": "UniProtKB:P33981",
  "term_id": "GO:0007059",
  "gene_symbol": "TTK",
  "term_label": "chromosome segregation"
}